{
  "gene_symbol": "MAZ",
  "gene": "UniProtKB:P56270",
  "gene_name": "Myc-associated zinc finger protein",
  "term_label": "regulation of transcription by RNA polymerase II",
  "term_id": "GO:0006357"
}